pyrimidine nucleobase transmembrane transport [GO:1904082] (biological process) Definition: The process in which pyrimidine is transported across a membrane. Subtypes: uracil transmembrane transport [GO:1903791] Sources: GOC:TermGenie, GO_REF:0000069 Relationships: is a type of pyrimidine nucleobase transport [GO:0015855]; is a type of pyrimidine-containing compound transmembrane transport [GO:0072531]